negative regulation of iron-sulfur-molybdenum cofactor assembly [GO:1900507] (biological process) Also known as: down regulation of FeMoco assembly, down regulation of FeMoco biosynthetic process, down regulation of iron molybdenum cofactor assembly, down regulation of iron molybdenum cofactor biosynthesis, down regulation of iron molybdenum cofactor biosynthetic process, down regulation of iron-sulfur-molybdenum cofactor assembly, down-regulation of FeMoco assembly, down-regulation of FeMoco biosynthetic process, down-regulation of iron molybdenum cofactor assembly, down-regulation of iron molybdenum cofactor biosynthesis, down-regulation of iron molybdenum cofactor biosynthetic process, down-regulation of iron-sulfur-molybdenum cofactor assembly, downregulation of FeMoco assembly, downregulation of FeMoco biosynthetic process, downregulation of iron molybdenum cofactor assembly, downregulation of iron molybdenum cofactor biosynthesis, downregulation of iron molybdenum cofactor biosynthetic process, downregulation of iron-sulfur-molybdenum cofactor assembly, inhibition of FeMoco assembly, inhibition of FeMoco biosynthetic process, inhibition of iron molybdenum cofactor assembly, inhibition of iron molybdenum cofactor biosynthesis, inhibition of iron molybdenum cofactor biosynthetic process, negative regulation of FeMoco assembly, negative regulation of FeMoco biosynthetic process, negative regulation of iron molybdenum cofactor assembly, negative regulation of iron molybdenum cofactor biosynthesis, negative regulation of iron molybdenum cofactor biosynthetic process, inhibition of iron-sulfur-molybdenum cofactor assembly Sources: GOC:TermGenie, GOC:mengo_curators Definition: Any process that stops, prevents or reduces the frequency, rate or extent of iron-sulfur-molybdenum cofactor assembly. Relationships: is a type of GO:1900506; is a type of negative regulation of iron-sulfur cluster assembly [GO:1903330]; RO_0002212 iron-sulfur-molybdenum cofactor assembly [GO:0044593]